{
  "gene": "UniProtKB:Q96PZ0",
  "gene_name": "Pseudouridylate synthase 7 homolog",
  "term_id": "GO:0009982",
  "term_label": "pseudouridine synthase activity",
  "gene_symbol": "PUS7"
}